{
  "gene": "UniProtKB:A0A0U1RQB9",
  "gene_symbol": "IGHD5-12",
  "gene_name": "Immunoglobulin heavy diversity 5-12 (Fragment)",
  "term_label": "Unknown cellular component",
  "term_id": "UNKNOWN:0003"
}